{
  "term_label": "epithelial structure maintenance",
  "gene_symbol": "FRAS1",
  "term_id": "GO:0010669",
  "gene": "UniProtKB:Q86XX4",
  "gene_name": "Extracellular matrix organizing protein FRAS1"
}